leading edge of lamellipodium [GO:0061851] (cellular component) Definition: That part of the lamellipodium which represents the distal part of the structure. Relationships: is a type of cell leading edge [GO:0031252]; is part of lamellipodium [GO:0030027] References: PMID:22339865